{
  "gene": "UniProtKB:Q9BXR0",
  "gene_name": "Queuine tRNA-ribosyltransferase catalytic subunit 1",
  "term_id": "UNKNOWN:0002",
  "term_label": "Unknown biological process",
  "gene_symbol": "QTRT1"
}